{
  "gene": "UniProtKB:P32856",
  "term_label": "presynaptic active zone membrane",
  "gene_name": "Syntaxin-2",
  "term_id": "GO:0048787",
  "gene_symbol": "STX2"
}